{
  "gene_name": "Neurogenic locus notch homolog protein 2",
  "term_label": "receptor complex",
  "term_id": "GO:0043235",
  "gene_symbol": "NOTCH2",
  "gene": "UniProtKB:Q04721"
}